{
  "gene_symbol": "ABCA7",
  "gene": "UniProtKB:Q8IZY2",
  "term_id": "GO:0042626",
  "gene_name": "Phospholipid-transporting ATPase ABCA7",
  "term_label": "ATPase-coupled transmembrane transporter activity"
}